{
  "gene_symbol": "PAX5",
  "gene": "UniProtKB:Q02548",
  "gene_name": "Paired box protein Pax-5",
  "term_id": "GO:0000981",
  "term_label": "DNA-binding transcription factor activity, RNA polymerase II-specific"
}